Golgi apparatus N-glycan diversification [GO:0016258] (biological process) Relationships: is a type of N-glycan processing [GO:0006491] Definition: The generation, in the Golgi apparatus, of side chain diversity from paucimannose mannose Man5GlcNAc2-Asn or Man3GlcNAc2-Asn N-glycans by specific glycosyltransferases and glycosidases. References: PMID:30858582, PMID:35536965 Also known as: N-glycan diversification